{
  "term_id": "GO:0001568",
  "term_label": "blood vessel development",
  "gene": "UniProtKB:Q13873",
  "gene_symbol": "BMPR2",
  "gene_name": "Bone morphogenetic protein receptor type-2"
}